chitin localization [GO:0006033] (biological process) Sources: GOC:ai Definition: A process in which chitin is transported to, or maintained in, a specific location. Also known as: chitin localisation, establishment and maintenance of chitin localization Relationships: is a type of polysaccharide localization [GO:0033037]